{
  "gene": "UniProtKB:Q96FV0",
  "gene_symbol": "LRRC46",
  "gene_name": "Leucine-rich repeat-containing protein 46",
  "term_id": "UNKNOWN:0002",
  "term_label": "Unknown biological process"
}